{
  "gene_name": "Fibrinogen silencer-binding protein",
  "gene_symbol": "FSBP",
  "gene": "UniProtKB:O95073",
  "term_label": "Unknown biological process",
  "term_id": "UNKNOWN:0002"
}